{
  "term_id": "GO:0004660",
  "gene": "UniProtKB:P49354",
  "gene_name": "Protein farnesyltransferase_geranylgeranyltransferase type-1 subunit alpha",
  "term_label": "protein farnesyltransferase activity",
  "gene_symbol": "FNTA"
}